{
  "term_label": "Unknown biological process",
  "gene_name": "Immunoglobulin superfamily member 3",
  "gene_symbol": "IGSF3",
  "term_id": "UNKNOWN:0002",
  "gene": "UniProtKB:O75054"
}